{
  "gene": "UniProtKB:Q96MD2",
  "gene_symbol": "KICS2",
  "term_label": "KICSTOR complex",
  "gene_name": "KICSTOR subunit 2",
  "term_id": "GO:0140007"
}